{
  "gene": "UniProtKB:P40855",
  "gene_symbol": "PEX19",
  "term_id": "GO:0033328",
  "term_label": "peroxisome membrane targeting sequence binding",
  "gene_name": "Peroxisomal biogenesis factor 19"
}